{
  "term_label": "Unknown biological process",
  "term_id": "UNKNOWN:0002",
  "gene_name": "Putative protein FAM47D",
  "gene_symbol": "FAM47DP",
  "gene": "UniProtKB:A6NHR8"
}